response to vitamin B6 [GO:0034516] (BP) Sources: GOC:mah, GOC:rph Definition: Any process that results in a change in state or activity of a cell or an organism (in terms of movement, secretion, enzyme production, gene expression, etc.) as a result of a vitamin B6 stimulus. Vitamin B6 encompasses pyridoxal, pyridoxamine and pyridoxine and the active form, pyridoxal phosphate. Relationships: is_a response to vitamin [GO:0033273]; is a type of response to nitrogen compound [GO:1901698]; is a type of response to oxygen-containing compound [GO:1901700] Subtypes: cellular response to vitamin B6 [GO:0071304]